endosome to plasma membrane transport vesicle [GO:0070381] (cellular component) Relationships: is a type of exocytic vesicle [GO:0070382] Definition: A transport vesicle that mediates transport from the endosome to the plasma membrane, and fuses with the plasma membrane to deliver lipids and membrane proteins to the plasma membrane and to release various cargo molecules, such as proteins or hormones, by exocytosis. Also known as: endosome to plasma membrane constitutive secretory pathway transport vesicle, endosome-plasma membrane transport vesicle References: PMID:10679016, PMID:12110576 Sources: GOC:kad, GOC:mah